{
  "gene_symbol": "KCNIP2",
  "term_id": "GO:0008076",
  "gene": "UniProtKB:Q9NS61",
  "term_label": "voltage-gated potassium channel complex",
  "gene_name": "Kv channel-interacting protein 2"
}